{
  "gene_name": "Proenkephalin-B",
  "term_id": "GO:0007218",
  "gene": "UniProtKB:P01213",
  "term_label": "neuropeptide signaling pathway",
  "gene_symbol": "PDYN"
}